{
  "gene_name": "ADP-ribosylation factor-like protein 13A",
  "term_label": "ciliary membrane",
  "gene_symbol": "ARL13A",
  "gene": "UniProtKB:Q5H913",
  "term_id": "GO:0060170"
}